{
  "term_id": "GO:0003700",
  "term_label": "DNA-binding transcription factor activity",
  "gene_symbol": "ZNF708",
  "gene_name": "Zinc finger protein 708",
  "gene": "UniProtKB:P17019"
}